glial limiting end-foot [GO:0097451] (cellular component) Definition: Terminal process of astrocyte that extends to the surface of the central nervous system. Together, glial limiting end-feet form the glial limiting membrane or glia limitans. Sources: NIF_Subcellular:sao181458425 Relationships: is a type of GO:0097450 Also known as: glial limiting endfoot